{
  "gene": "UniProtKB:Q4G0M1",
  "gene_symbol": "ERFE",
  "gene_name": "Erythroferrone",
  "term_id": "GO:0045721",
  "term_label": "negative regulation of gluconeogenesis"
}